{
  "term_label": "structural constituent of chromatin",
  "gene_name": "Histone H2A.Z",
  "gene": "UniProtKB:P0C0S5",
  "term_id": "GO:0030527",
  "gene_symbol": "H2AZ1"
}